{
  "gene_name": "Semaphorin-6C",
  "gene_symbol": "SEMA6C",
  "term_label": "semaphorin receptor binding",
  "gene": "UniProtKB:Q9H3T2",
  "term_id": "GO:0030215"
}